{
  "term_label": "cellular response to lipopolysaccharide",
  "gene_symbol": "IL1A",
  "gene_name": "Interleukin-1 alpha",
  "term_id": "GO:0071222",
  "gene": "UniProtKB:P01583"
}